{
  "term_label": "DNA-binding transcription factor activity, RNA polymerase II-specific",
  "gene": "UniProtKB:O00716",
  "gene_name": "Transcription factor E2F3",
  "term_id": "GO:0000981",
  "gene_symbol": "E2F3"
}